{
  "gene_symbol": "PIK3R3",
  "gene": "UniProtKB:Q92569",
  "term_id": "GO:0008286",
  "gene_name": "Phosphatidylinositol 3-kinase regulatory subunit gamma",
  "term_label": "insulin receptor signaling pathway"
}